{
  "gene_name": "Unconventional myosin-Va",
  "gene_symbol": "MYO5A",
  "gene": "UniProtKB:Q9Y4I1",
  "term_label": "actin filament binding",
  "term_id": "GO:0051015"
}